{
  "gene": "UniProtKB:P02545",
  "term_label": "structural constituent of cytoskeleton",
  "gene_name": "Prelamin-A_C",
  "term_id": "GO:0005200",
  "gene_symbol": "LMNA"
}